{
  "gene": "UniProtKB:Q9UK55",
  "gene_name": "Protein Z-dependent protease inhibitor",
  "term_label": "Unknown biological process",
  "term_id": "UNKNOWN:0002",
  "gene_symbol": "SERPINA10"
}